{
  "term_label": "amino acid metabolic process",
  "term_id": "GO:0006520",
  "gene_name": "1-aminocyclopropane-1-carboxylate synthase-like protein 1",
  "gene_symbol": "ACCS",
  "gene": "UniProtKB:Q96QU6"
}